{
  "gene": "UniProtKB:Q5VST6",
  "term_label": "negative regulation of protein localization to microtubule",
  "gene_symbol": "ABHD17B",
  "gene_name": "Alpha_beta hydrolase domain-containing protein 17B",
  "term_id": "GO:1902817"
}